{
  "gene_symbol": "SIGLEC11",
  "gene": "UniProtKB:Q96RL6",
  "term_label": "plasma membrane",
  "gene_name": "Sialic acid-binding Ig-like lectin 11",
  "term_id": "GO:0005886"
}